viral replication complex formation and maintenance [GO:0046786] (biological process) Relationships: is a type of viral process [GO:0016032]; is part of viral genome replication [GO:0019079] Sources: ISBN:0781718325 Definition: The process of organizing and assembling viral replication proteins in preparation for viral replication.